{
  "gene_name": "POTE ankyrin domain family member J",
  "term_id": "GO:0005737",
  "gene_symbol": "POTEJ",
  "term_label": "cytoplasm",
  "gene": "UniProtKB:P0CG39"
}